{
  "term_id": "UNKNOWN:0003",
  "gene_name": "Protein FAM229A",
  "gene_symbol": "FAM229A",
  "gene": "UniProtKB:H3BQW9",
  "term_label": "Unknown cellular component"
}